{
  "gene": "UniProtKB:Q9UDR5",
  "gene_symbol": "AASS",
  "gene_name": "Alpha-aminoadipic semialdehyde synthase, mitochondrial",
  "term_id": "GO:0005737",
  "term_label": "cytoplasm"
}